{
  "gene_name": "Secretagogin",
  "gene": "UniProtKB:O76038",
  "gene_symbol": "SCGN",
  "term_label": "Unknown biological process",
  "term_id": "UNKNOWN:0002"
}